positive regulation of release of sequestered calcium ion into cytosol [GO:0051281] (biological process) Definition: Any process that activates or increases the frequency, rate or extent of the release into the cytosolic compartment of calcium ions sequestered in the endoplasmic reticulum or mitochondria. Sources: GOC:ai Relationships: is a type of regulation of release of sequestered calcium ion into cytosol [GO:0051279]; is a type of GO:1904427; RO_0002213 release of sequestered calcium ion into cytosol [GO:0051209] Also known as: positive regulation of calcium ion (Ca2+) mobilization, positive regulation of calcium mobilization, positive regulation of cytoplasmic release of sequestered calcium ion (Ca2+), positive regulation of cytoplasmic release of stored calcium ion (Ca2+), positive regulation of release of sequestered calcium ion (Ca2+), positive regulation of release of sequestered calcium ion into cytoplasm, positive regulation of release of stored calcium ion (Ca2+), positive regulation of release of stored calcium ion (Ca2+) into cytoplasm, positive regulation of cytosolic release of sequestered calcium ion (Ca2+), positive regulation of cytosolic release of stored calcium ion (Ca2+), positive regulation of release of stored calcium ion (Ca2+) into cytosol, up regulation of release of sequestered calcium ion into cytosol, up-regulation of release of sequestered calcium ion into cytosol, upregulation of release of sequestered calcium ion into cytosol, activation of release of sequestered calcium ion into cytosol, stimulation of release of sequestered calcium ion into cytosol